{
  "term_id": "GO:0070374",
  "gene": "UniProtKB:O60658",
  "gene_symbol": "PDE8A",
  "term_label": "positive regulation of ERK1 and ERK2 cascade",
  "gene_name": "High affinity cAMP-specific and IBMX-insensitive 3',5'-cyclic phosphodiesterase 8A"
}